{
  "term_id": "GO:0072659",
  "gene_name": "EH domain-containing protein 3",
  "gene": "UniProtKB:Q9NZN3",
  "gene_symbol": "EHD3",
  "term_label": "protein localization to plasma membrane"
}